{
  "gene_symbol": "EPHB4",
  "gene_name": "Ephrin type-B receptor 4",
  "gene": "UniProtKB:P54760",
  "term_id": "GO:0004714",
  "term_label": "transmembrane receptor protein tyrosine kinase activity"
}